{
  "term_label": "protein deneddylation",
  "gene_name": "COP9 signalosome complex subunit 2",
  "term_id": "GO:0000338",
  "gene": "UniProtKB:P61201",
  "gene_symbol": "COPS2"
}